{
  "term_label": "microtubule cytoskeleton organization",
  "gene_symbol": "MAPT",
  "gene": "UniProtKB:P10636",
  "gene_name": "Microtubule-associated protein tau",
  "term_id": "GO:0000226"
}